{
  "gene_name": "Probable inactive ribonuclease-like protein 12",
  "term_label": "defense response to Gram-positive bacterium",
  "gene_symbol": "RNASE12",
  "gene": "UniProtKB:Q5GAN4",
  "term_id": "GO:0050830"
}